{
  "term_label": "protein polyubiquitination",
  "term_id": "GO:0000209",
  "gene": "UniProtKB:Q9UKT5",
  "gene_name": "F-box only protein 4",
  "gene_symbol": "FBXO4"
}